{
  "gene_symbol": "AKT1",
  "term_id": "GO:0004674",
  "gene_name": "RAC-alpha serine_threonine-protein kinase",
  "term_label": "protein serine/threonine kinase activity",
  "gene": "UniProtKB:P31749"
}